{
  "gene": "UniProtKB:O43593",
  "gene_name": "Lysine-specific demethylase hairless",
  "term_id": "GO:0031490",
  "term_label": "chromatin DNA binding",
  "gene_symbol": "HR"
}